{
  "gene_name": "Inactive tyrosine-protein kinase PRAG1",
  "term_id": "GO:2000145",
  "gene_symbol": "PRAG1",
  "gene": "UniProtKB:Q86YV5",
  "term_label": "regulation of cell motility"
}